membrane fusion priming complex [GO:0120124] (cellular component) Also known as: GATE-16 complex, LMA1 complex Relationships: is a type of protein-containing complex [GO:0032991] Definition: A protein complex that primes vacuolar or vesicular membranes for fusion with other intracellular membranes, by promoting the dissociation of cis-SNARE complexes. References: PMID:9015301 Sources: GOC:lnp